{
  "gene": "UniProtKB:Q96S21",
  "gene_name": "Ras-related protein Rab-40C",
  "term_id": "GO:0003924",
  "term_label": "GTPase activity",
  "gene_symbol": "RAB40C"
}